{
  "term_id": "GO:0070990",
  "gene_symbol": "SNRPN",
  "gene": "UniProtKB:P63162",
  "gene_name": "Small nuclear ribonucleoprotein-associated protein N",
  "term_label": "snRNP binding"
}